activated CD8-positive, alpha-beta T cell apoptotic process [GO:1905397] (biological process) Definition: Any apoptotic process in an activated CD8-positive, alpha-beta T cell. Also known as: activated CD8-positive, alpha-beta T lymphocyte apoptotic process, activated CD8-positive, alpha-beta T-cell apoptotic process, activated CD8-positive, alpha-beta T-lymphocyte apoptotic process, activated CD8-positive, alpha-beta T cell apoptosis, activated CD8-positive, alpha-beta T lymphocyte apoptosis, activated CD8-positive, alpha-beta T-cell apoptosis, activated CD8-positive, alpha-beta T-lymphocyte apoptosis Relationships: is a type of GO:0070231 References: PMID:24187568 Sources: GOC:TermGenie, GO_REF:0000085 Regulation: regulated by regulation of activated CD8-positive, alpha-beta T cell apoptotic process [GO:1905402]; negatively regulated by negative regulation of activated CD8-positive, alpha-beta T cell apoptotic process [GO:1905403]; positively regulated by positive regulation of activated CD8-positive, alpha-beta T cell apoptotic process [GO:1905404]